{
  "gene_name": "RILP-like protein 2",
  "gene": "UniProtKB:Q969X0",
  "term_label": "ciliary basal body",
  "gene_symbol": "RILPL2",
  "term_id": "GO:0036064"
}